{
  "gene_symbol": "DEFA5",
  "gene_name": "Defensin alpha 5",
  "gene": "UniProtKB:Q01523",
  "term_label": "defense response to Gram-negative bacterium",
  "term_id": "GO:0050829"
}